{
  "gene_name": "Sarcoplasmic_endoplasmic reticulum calcium ATPase 2",
  "gene_symbol": "ATP2A2",
  "gene": "UniProtKB:P16615",
  "term_id": "GO:0000045",
  "term_label": "autophagosome assembly"
}